triglyceride-rich lipoprotein particle clearance [GO:0071830] (biological process) Subtypes: chylomicron remnant clearance [GO:0034382], intermediate-density lipoprotein particle clearance [GO:0071831] Relationships: is a type of plasma lipoprotein particle clearance [GO:0034381] Definition: The process in which a triglyceride-rich lipoprotein particle is removed from the blood via receptor-mediated endocytosis and its constituent parts degraded. Sources: GOC:BHF